{
  "gene_name": "Syntaxin-2",
  "gene_symbol": "STX2",
  "term_label": "SNARE binding",
  "gene": "UniProtKB:P32856",
  "term_id": "GO:0000149"
}